{
  "term_id": "GO:2000562",
  "term_label": "negative regulation of CD4-positive, alpha-beta T cell proliferation",
  "gene_name": "Galectin-9C",
  "gene_symbol": "LGALS9C",
  "gene": "UniProtKB:Q6DKI2"
}